{
  "term_label": "actin filament bundle",
  "gene_name": "Plastin-2",
  "gene_symbol": "LCP1",
  "term_id": "GO:0032432",
  "gene": "UniProtKB:P13796"
}